symbiont-mediated suppression of host cell wall biogenesis [GO:0039636] (biological process) Sources: GOC:bf, GOC:bm, GOC:jl Definition: Any process in which a virus stops, prevents, or reduces the frequency, rate or extent of cell wall biogenesis in the host organism. Cell wall biogenesis includes the biosynthesis of constituent macromolecules, and the assembly and arrangement of these constituent parts. Relationships: is_a symbiont-mediated perturbation of host cellular process [GO:0044068] Also known as: suppression by virus of host cell wall biogenesis